response to bismuth [GO:0072700] (BP) Also known as: response to bismuth ion Subtypes: cellular response to bismuth [GO:0072701] Sources: GOC:mah Definition: Any process that results in a change in state or activity of a cell or an organism (in terms of movement, secretion, enzyme production, gene expression, etc.) as a result of a bismuth (Bi) stimulus. Relationships: is a type of response to chemical [GO:0042221]